{
  "gene_symbol": "PTHLH",
  "term_id": "GO:0032330",
  "gene": "UniProtKB:P12272",
  "gene_name": "Parathyroid hormone-related protein",
  "term_label": "regulation of chondrocyte differentiation"
}